{
  "term_id": "GO:0007420",
  "gene_symbol": "SOX12",
  "term_label": "brain development",
  "gene_name": "Transcription factor SOX-12",
  "gene": "UniProtKB:O15370"
}